neuron projection fasciculation [GO:0106030] (biological process) Definition: The collection of neuronal projections into a bundle of rods, known as a fascicle. References: PMID:12761826 Sources: GOC:aruk, GOC:bc. Relationships: is a type of GO:0031175 Subtypes: axonal fasciculation [GO:0007413]